{
  "term_label": "cytokine-mediated signaling pathway",
  "term_id": "GO:0019221",
  "gene_name": "Suppressor of cytokine signaling 4",
  "gene": "UniProtKB:Q8WXH5",
  "gene_symbol": "SOCS4"
}